{
  "gene": "UniProtKB:Q6UXB4",
  "term_id": "GO:0006955",
  "term_label": "immune response",
  "gene_name": "C-type lectin domain family 4 member G",
  "gene_symbol": "CLEC4G"
}